{
  "term_label": "proteasome-mediated ubiquitin-dependent protein catabolic process",
  "gene_symbol": "RNF4",
  "gene": "UniProtKB:P78317",
  "gene_name": "E3 ubiquitin-protein ligase RNF4",
  "term_id": "GO:0043161"
}